{
  "term_label": "synaptic vesicle lumen acidification",
  "gene_symbol": "ATP6V1G1",
  "gene": "UniProtKB:O75348",
  "gene_name": "V-type proton ATPase subunit G 1",
  "term_id": "GO:0097401"
}